{
  "term_label": "regulation of cell adhesion",
  "term_id": "GO:0030155",
  "gene_symbol": "CYTIP",
  "gene": "UniProtKB:O60759",
  "gene_name": "Cytohesin-interacting protein"
}